{
  "gene": "UniProtKB:O60478",
  "gene_name": "Integral membrane protein GPR137B",
  "gene_symbol": "GPR137B",
  "term_id": "UNKNOWN:0001",
  "term_label": "Unknown molecular function"
}